L-aspartate import across plasma membrane [GO:0140009] (biological process) Relationships: is a type of GO:0070778; is a type of amino acid import across plasma membrane [GO:0089718] References: PMID:7914198 Sources: GO_REF:0000069 Definition: The directed movement of L-aspartate from outside of a cell, across the plasma membrane and into the cytosol.